{
  "term_label": "single-stranded telomeric DNA binding",
  "gene": "UniProtKB:P27694",
  "gene_name": "Replication protein A 70 kDa DNA-binding subunit",
  "term_id": "GO:0043047",
  "gene_symbol": "RPA1"
}